{
  "term_label": "DNA translocase activity",
  "gene_name": "DNA repair and recombination protein RAD54-like",
  "gene_symbol": "RAD54L",
  "gene": "UniProtKB:Q92698",
  "term_id": "GO:0015616"
}